{
  "term_label": "cell-cell adhesion",
  "gene_name": "Plakophilin-2",
  "term_id": "GO:0098609",
  "gene_symbol": "PKP2",
  "gene": "UniProtKB:Q99959"
}